{
  "gene_name": "Adenylate cyclase type 9",
  "term_label": "adenylate cyclase activity",
  "gene": "UniProtKB:O60503",
  "term_id": "GO:0004016",
  "gene_symbol": "ADCY9"
}